{
  "gene_name": "Ras GTPase-activating protein-binding protein 1",
  "term_id": "GO:0003729",
  "term_label": "mRNA binding",
  "gene": "UniProtKB:Q13283",
  "gene_symbol": "G3BP1"
}